{
  "term_id": "GO:0005815",
  "gene": "UniProtKB:P41002",
  "gene_name": "Cyclin-F",
  "gene_symbol": "CCNF",
  "term_label": "microtubule organizing center"
}